mRNA cleavage and polyadenylation specificity factor complex assembly [GO:0110105] (biological process) References: PMID:27401558 Sources: GOC:mah Definition: The aggregation, arrangement and bonding together of a set of components to form the mRNA cleavage and polyadenylation specificity factor complex. Relationships: is a type of protein-containing complex assembly [GO:0065003]; is part of RNA 3'-end processing [GO:0031123]